{
  "gene": "UniProtKB:Q9Y5B8",
  "term_label": "Unknown molecular function",
  "gene_symbol": "NME7",
  "gene_name": "Nucleoside diphosphate kinase 7",
  "term_id": "UNKNOWN:0001"
}